immune response-regulating signaling pathway [GO:0002764] (biological process) Definition: The cascade of processes by which a signal interacts with a receptor, causing a change in the level or activity of a second messenger or other downstream target, and ultimately leading to the activation, perpetuation, or inhibition of an immune response. Also known as: immune response-regulating signalling pathway Relationships: is a type of signal transduction [GO:0007165]; is a type of regulation of immune response [GO:0050776] Subtypes: immune response-activating signaling pathway [GO:0002757], immune response-inhibiting signal transduction [GO:0002765], immune response-regulating cell surface receptor signaling pathway [GO:0002768] References: PMID:15771571 Sources: GOC:add, ISBN:0781735149